regulation of microtubule polymerization [GO:0031113] (biological process) Definition: Any process that modulates the frequency, rate or extent of microtubule polymerization. Relationships: is a type of regulation of microtubule polymerization or depolymerization [GO:0031110]; is a type of regulation of protein polymerization [GO:0032271]; is a type of regulation of supramolecular fiber organization [GO:1902903]; regulates microtubule polymerization [GO:0046785] Subtypes: GO:0010968, GO:0031115, positive regulation of microtubule polymerization [GO:0031116] Sources: GOC:mah